{
  "gene_name": "Protein EFR3 homolog B",
  "term_label": "Unknown molecular function",
  "term_id": "UNKNOWN:0001",
  "gene": "UniProtKB:Q9Y2G0",
  "gene_symbol": "EFR3B"
}